{
  "gene_symbol": "ZBTB1",
  "gene": "UniProtKB:Q9Y2K1",
  "gene_name": "Zinc finger and BTB domain-containing protein 1",
  "term_label": "regulation of cytokine production",
  "term_id": "GO:0001817"
}